{
  "gene_symbol": "NUP54",
  "gene": "UniProtKB:Q7Z3B4",
  "term_id": "GO:0017056",
  "gene_name": "Nucleoporin p54",
  "term_label": "structural constituent of nuclear pore"
}